platelet-derived growth factor receptor activity [GO:0005017] (molecular function) Relationships: is_a transmembrane receptor protein tyrosine kinase activity [GO:0004714]; is part of cellular response to platelet-derived growth factor stimulus [GO:0036120]; is part of platelet-derived growth factor receptor signaling pathway [GO:0048008]; has part platelet-derived growth factor binding [GO:0048407] Note: Note that this term represents an activity and not a gene product, and should only be used when the receptor binds the ligand PDGF. For receptors that bind other growth factors, consider annotating to other terms under 'transmembrane signaling receptor activity ; GO:0004888. Sources: GOC:mah Also known as: PDGF receptor activity, PDGF-activated receptor activity, PDGFR activity, platelet-derived growth factor-activated receptor activity Definition: Combining with platelet-derived growth factor receptor ligand and transmitting the signal across the plasma membrane to initiate a change in cell activity. Subtypes: GO:0005018, platelet-derived growth factor beta-receptor activity [GO:0005019]